prominosome [GO:0071914] (cellular component) Relationships: is a type of GO:1903561 Also known as: prominin-containing extracellular membrane vesicle Definition: An extracellular membrane-bounded vesicle that contains prominin proteins (in mouse Prom1/CD33 or Prom2) and are found in body fluids including ventricular fluid, saliva, urine and seminal fluid. In the ventricular fluid of the developing mouse brain two major classes of these particles have been observed (P2 particles of 500-1000 nm and P4 particles of 50-80 nm) which likely originate from microvilli, primary cilia and/or the midbody of neuroepithelial cells. The physiological role is not known. References: PMID:15976444, PMID:17109118, PMID:17283184 Sources: GOC:vesicles